nucleobase-containing compound transport [GO:0015931] (biological process) Also known as: nucleobase, nucleoside, nucleotide and nucleic acid transport Subtypes: GO:0006862, nucleotide-sulfate transport [GO:0015715], GO:0015780, nucleoside transport [GO:0015858], GO:0015869, coenzyme A transport [GO:0015880], fatty-acyl-CoA transport [GO:0015916], nucleic acid transport [GO:0050657] Definition: The directed movement of nucleobases, nucleosides, nucleotides and nucleic acids, into, out of or within a cell, or between cells, by means of some agent such as a transporter or pore. Relationships: is a type of nitrogen compound transport [GO:0071705] Sources: GOC:ai Regulation: regulated by regulation of nucleobase-containing compound transport [GO:0032239]; negatively regulated by negative regulation of nucleobase-containing compound transport [GO:0032240]; positively regulated by positive regulation of nucleobase-containing compound transport [GO:0032241]